{
  "gene": "UniProtKB:Q8IU57",
  "gene_name": "Interferon lambda receptor 1",
  "term_id": "GO:0004896",
  "term_label": "cytokine receptor activity",
  "gene_symbol": "IFNLR1"
}